{
  "gene_symbol": "CD1A",
  "term_id": "GO:0030884",
  "gene": "UniProtKB:P06126",
  "gene_name": "T-cell surface glycoprotein CD1a",
  "term_label": "exogenous lipid antigen binding"
}